regulation of DNA-templated DNA replication [GO:0090329] (biological process) Subtypes: GO:0030174, regulation of DNA endoreduplication [GO:0032875], GO:0033262, regulation of mitochondrial DNA replication [GO:0090296], GO:1902681, negative regulation of DNA-templated DNA replication [GO:2000104], GO:2000105, GO:2000621 Relationships: is_a regulation of DNA replication [GO:0006275]; regulates DNA-templated DNA replication [GO:0006261] Also known as: regulation of DNA-dependent DNA replication Definition: Any process that modulates the rate, frequency, or extent of DNA-templated DNA replication, the process in which new strands of DNA are synthesized. Sources: GOC:dph, GOC:tb